{
  "gene_symbol": "TNNI2",
  "gene_name": "Troponin I, fast skeletal muscle",
  "term_id": "GO:0005861",
  "term_label": "troponin complex",
  "gene": "UniProtKB:P48788"
}